{
  "gene_symbol": "PEX10",
  "gene": "UniProtKB:O60683",
  "term_id": "GO:0005778",
  "term_label": "peroxisomal membrane",
  "gene_name": "Peroxisome biogenesis factor 10"
}